UAG codon-amino acid adaptor activity [GO:0033412] (molecular function) Also known as: TAG codon-amino acid adaptor activity Relationships: is a type of triplet codon-amino acid adaptor activity [GO:0030533] Definition: A triplet codon-amino acid adaptor activity that recognizes a UAG codon. Note: Note that in the standard genetic code, TAG is a stop codon (amber) and is not normally read by a tRNA. Sources: GOC:mah